{
  "gene_name": "Solute carrier family 22 member 25",
  "term_label": "Unknown molecular function",
  "gene_symbol": "SLC22A25",
  "term_id": "UNKNOWN:0001",
  "gene": "UniProtKB:Q6T423"
}